{
  "term_label": "nucleus",
  "gene_name": "RNA-binding protein FXR2",
  "gene": "UniProtKB:P51116",
  "term_id": "GO:0005634",
  "gene_symbol": "FXR2"
}